{
  "gene_name": "Immunoglobulin lambda variable 7-43",
  "gene": "UniProtKB:P04211",
  "term_label": "immunoglobulin complex",
  "term_id": "GO:0019814",
  "gene_symbol": "IGLV7-43"
}